positive regulation of lymphoid progenitor cell differentiation [GO:1905458] (biological process) Relationships: is a type of positive regulation of hematopoietic progenitor cell differentiation [GO:1901534]; is a type of regulation of lymphoid progenitor cell differentiation [GO:1905456]; positively regulates lymphoid progenitor cell differentiation [GO:0002320] Subtypes: GO:2000176, GO:2000975 Also known as: up regulation of lymphoid progenitor cell differentiation, up-regulation of lymphoid progenitor cell differentiation, upregulation of lymphoid progenitor cell differentiation, activation of lymphoid progenitor cell differentiation Definition: Any process that activates or increases the frequency, rate or extent of lymphoid progenitor cell differentiation. References: PMID:27010503 Sources: GOC:TermGenie, GO_REF:0000058